{
  "gene": "UniProtKB:Q5EBL2",
  "gene_name": "Zinc finger protein 628",
  "term_label": "DNA-binding transcription factor activity, RNA polymerase II-specific",
  "gene_symbol": "ZNF628",
  "term_id": "GO:0000981"
}